{
  "gene_symbol": "MARK2",
  "term_label": "tau-protein kinase activity",
  "gene": "UniProtKB:Q7KZI7",
  "gene_name": "Serine_threonine-protein kinase MARK2",
  "term_id": "GO:0050321"
}